{
  "term_id": "GO:0005685",
  "gene_name": "U1 small nuclear ribonucleoprotein A",
  "gene": "UniProtKB:P09012",
  "term_label": "U1 snRNP",
  "gene_symbol": "SNRPA"
}